{
  "gene_name": "R3H domain-containing protein 1",
  "term_id": "UNKNOWN:0002",
  "term_label": "Unknown biological process",
  "gene": "UniProtKB:Q15032",
  "gene_symbol": "R3HDM1"
}